regulation of podocyte apoptotic process [GO:1904633] (BP) Also known as: regulation of glomerular podocyte apoptotic process, regulation of glomerular visceral epithelial cell apoptotic process, regulation of glomerular podocyte apoptosis, regulation of glomerular visceral epithelial cell apoptosis, regulation of podocyte apoptosis Subtypes: negative regulation of podocyte apoptotic process [GO:1904634], positive regulation of podocyte apoptotic process [GO:1904635] Definition: Any process that modulates the frequency, rate or extent of glomerular visceral epithelial cell apoptotic process. References: PMID:23692924 Sources: GOC:TermGenie, GO_REF:0000058 Relationships: is a type of GO:1904035; regulates podocyte apoptotic process [GO:1903210]